{
  "gene": "UniProtKB:Q71RG6",
  "gene_name": "Putative chemokine-related protein FP248",
  "term_id": "UNKNOWN:0003",
  "gene_symbol": "FP248",
  "term_label": "Unknown cellular component"
}